renal potassium excretion [GO:0036359] (biological process) Definition: The elimination of potassium ions from peritubular capillaries (or surrounding hemolymph in invertebrates) into the renal tubules to be incorporated subsequently into the urine. References: PMID:15034090, PMID:25287933 Sources: GOC:gap Also known as: renal K(+) excretion, renal K+ elimination, renal potassium ion excretion Relationships: is a type of renal tubular secretion [GO:0097254]